{
  "gene_name": "WD repeat, SAM and U-box domain-containing protein 1",
  "gene": "UniProtKB:Q8N9V3",
  "term_label": "Unknown biological process",
  "gene_symbol": "WDSUB1",
  "term_id": "UNKNOWN:0002"
}